{
  "term_label": "smoothened signaling pathway",
  "gene": "UniProtKB:Q8N158",
  "gene_symbol": "GPC2",
  "term_id": "GO:0007224",
  "gene_name": "Glypican-2"
}